{
  "gene_name": "Lipid droplet assembly factor 1",
  "term_label": "Unknown biological process",
  "term_id": "UNKNOWN:0002",
  "gene": "UniProtKB:Q96B96",
  "gene_symbol": "LDAF1"
}